N-terminal peptidyl-proline dimethylation [GO:0018016] (biological process) Relationships: is a type of GO:0035568 Sources: RESID:AA0066 Definition: The methylation of the N-terminal proline of proteins to form the derivative N,N-dimethyl-L-proline.